post-embryonic root morphogenesis [GO:0010101] (biological process) Relationships: is a type of GO:0010015; is a type of GO:0090697; is part of post-embryonic root development [GO:0048528] Definition: The process in which the anatomical structures of the post-embryonic root are generated and organized. The post-embryonic root is the root formed after the embryonic phase has been completed. Sources: GOC:tb Subtypes: lateral root morphogenesis [GO:0010102]